{
  "gene": "UniProtKB:Q96B97",
  "term_label": "Unknown cellular component",
  "gene_name": "SH3 domain-containing kinase-binding protein 1",
  "term_id": "UNKNOWN:0003",
  "gene_symbol": "SH3KBP1"
}